regulation of microvillus length [GO:0032532] (biological process) Subtypes: GO:0032533, negative regulation of microvillus length [GO:1903982], positive regulation of microvillus length [GO:1903983] Definition: A process that modulates the length of a microvillus. Relationships: is a type of regulation of microvillus organization [GO:0032530]; is a type of regulation of cell projection size [GO:0032536] Sources: GOC:mah